{
  "gene_name": "HMG box transcription factor BBX",
  "gene": "UniProtKB:Q8WY36",
  "gene_symbol": "BBX",
  "term_id": "GO:0000981",
  "term_label": "DNA-binding transcription factor activity, RNA polymerase II-specific"
}